{
  "term_id": "UNKNOWN:0002",
  "term_label": "Unknown biological process",
  "gene_symbol": "NXPH4",
  "gene": "UniProtKB:O95158",
  "gene_name": "Neurexophilin-4"
}